{
  "gene_name": "Period circadian protein homolog 3",
  "gene": "UniProtKB:P56645",
  "term_id": "GO:0032922",
  "term_label": "circadian regulation of gene expression",
  "gene_symbol": "PER3"
}